{
  "gene_name": "Histone acetyltransferase type B catalytic subunit",
  "gene_symbol": "HAT1",
  "term_id": "GO:0010485",
  "term_label": "histone H4 acetyltransferase activity",
  "gene": "UniProtKB:O14929"
}